{
  "term_id": "GO:0000287",
  "gene_name": "Bifunctional epoxide hydrolase 2",
  "term_label": "magnesium ion binding",
  "gene": "UniProtKB:P34913",
  "gene_symbol": "EPHX2"
}